{
  "term_id": "GO:0032217",
  "gene_symbol": "ABCG2",
  "term_label": "riboflavin transmembrane transporter activity",
  "gene_name": "Broad substrate specificity ATP-binding cassette transporter ABCG2",
  "gene": "UniProtKB:Q9UNQ0"
}